{
  "gene_symbol": "KLK2",
  "term_id": "GO:0030141",
  "term_label": "secretory granule",
  "gene": "UniProtKB:P20151",
  "gene_name": "Kallikrein-2"
}